{
  "term_id": "GO:0018279",
  "gene_name": "Oligosaccharyltransferase complex subunit OSTC",
  "gene": "UniProtKB:Q9NRP0",
  "gene_symbol": "OSTC",
  "term_label": "protein N-linked glycosylation via asparagine"
}